{
  "term_label": "signal peptide processing",
  "gene_name": "Signal peptidase complex subunit 2",
  "term_id": "GO:0006465",
  "gene_symbol": "SPCS2",
  "gene": "UniProtKB:Q15005"
}